{
  "term_id": "GO:0060271",
  "gene": "UniProtKB:Q2M329",
  "term_label": "cilium assembly",
  "gene_symbol": "CFAP184",
  "gene_name": "Coiled-coil domain-containing protein 96"
}